steryl-sulfatase activity [GO:0004773] (molecular function) Definition: Catalysis of the reaction: 3-beta-hydroxyandrost-5-en-17-one 3-sulfate + H2O = 3-beta-hydroxyandrost-5-en-17-one + sulfate. Relationships: is a type of sulfuric ester hydrolase activity [GO:0008484] Sources: EC:3.1.6.2 Also known as: steryl-sulphatase activity, 3-beta-hydroxysteroid sulfate sulfatase activity, arylsulfatase C activity, dehydroepiandrosterone sulfatase activity, dehydroepiandrosterone sulfate sulfatase activity, phenolic steroid sulfatase activity, pregnenolone sulfatase activity, steroid 3-sulfatase activity, steroid sulfatase activity, steroid sulfate sulfohydrolase activity, sterol sulfatase activity, steryl-sulfate sulfohydrolase activity